{
  "gene_name": "Solute carrier family 22 member 4",
  "term_id": "GO:0015651",
  "gene_symbol": "SLC22A4",
  "gene": "UniProtKB:Q9H015",
  "term_label": "quaternary ammonium group transmembrane transporter activity"
}